{
  "gene_symbol": "HNF4A",
  "gene_name": "Hepatocyte nuclear factor 4-alpha",
  "term_label": "Unknown cellular component",
  "gene": "UniProtKB:P41235",
  "term_id": "UNKNOWN:0003"
}